positive regulation of hydrogen peroxide-mediated programmed cell death [GO:1901300] (BP) Definition: Any process that activates or increases the frequency, rate or extent of hydrogen peroxide-mediated programmed cell death. Subtypes: positive regulation of intrinsic apoptotic signaling pathway in response to hydrogen peroxide [GO:1903752] Sources: GOC:BHF, GOC:TermGenie Also known as: up regulation of hydrogen peroxide-mediated programmed cell death, up-regulation of hydrogen peroxide-mediated programmed cell death, upregulation of hydrogen peroxide-mediated programmed cell death, activation of hydrogen peroxide-mediated programmed cell death Relationships: is_a positive regulation of programmed cell death [GO:0043068]; is a type of regulation of hydrogen peroxide-mediated programmed cell death [GO:1901298]; positively regulates hydrogen peroxide-mediated programmed cell death [GO:0010421]